{
  "gene_symbol": "VPS41",
  "term_id": "GO:0034058",
  "gene": "UniProtKB:P49754",
  "term_label": "endosomal vesicle fusion",
  "gene_name": "Vacuolar protein sorting-associated protein 41 homolog"
}